{
  "gene_name": "DNA-binding protein RFXANK",
  "gene_symbol": "RFXANK",
  "term_label": "positive regulation of transcription by RNA polymerase II",
  "term_id": "GO:0045944",
  "gene": "UniProtKB:O14593"
}